[choline trimethylamine-lyase]-activating enzyme activity [GO:0140111] (molecular function) Relationships: is a type of glycyl-radical enzyme activating activity [GO:0043364] References: PMID:24854437 Definition: Catalyzes the activation of choline trimethylamine-lyase by generation of an organic free radical on a glycine residue via a homolytic cleavage of S-adenosyl-L-methionine (SAM).